{
  "term_id": "GO:0000122",
  "gene_symbol": "TGIF2LX",
  "term_label": "negative regulation of transcription by RNA polymerase II",
  "gene": "UniProtKB:Q8IUE1",
  "gene_name": "Homeobox protein TGIF2LX"
}